{
  "gene": "UniProtKB:Q96SQ5",
  "term_label": "DNA-binding transcription factor activity, RNA polymerase II-specific",
  "term_id": "GO:0000981",
  "gene_name": "Zinc finger protein 587",
  "gene_symbol": "ZNF587"
}